{
  "term_label": "regulation of transcription by RNA polymerase II",
  "gene": "UniProtKB:Q6NSZ9",
  "term_id": "GO:0006357",
  "gene_symbol": "ZSCAN25",
  "gene_name": "Zinc finger and SCAN domain-containing protein 25"
}